{
  "term_id": "GO:0007018",
  "gene_symbol": "KIF2A",
  "term_label": "microtubule-based movement",
  "gene": "UniProtKB:O00139",
  "gene_name": "Kinesin-like protein KIF2A"
}